{
  "gene_symbol": "BCL2A1",
  "gene_name": "Bcl-2-related protein A1",
  "term_label": "intrinsic apoptotic signaling pathway in response to DNA damage",
  "gene": "UniProtKB:Q16548",
  "term_id": "GO:0008630"
}